{
  "term_label": "Unknown cellular component",
  "gene": "UniProtKB:Q9HCE3",
  "term_id": "UNKNOWN:0003",
  "gene_symbol": "ZNF532",
  "gene_name": "Zinc finger protein 532"
}